{
  "gene_symbol": "VGF",
  "term_id": "GO:0005615",
  "gene": "UniProtKB:O15240",
  "term_label": "extracellular space",
  "gene_name": "Neurosecretory protein VGF"
}